calcium-dependent carbohydrate binding [GO:0120153] (molecular function) Relationships: is a type of carbohydrate binding [GO:0030246] Definition: Binding to a carbohydrate in the presence of calcium. References: PMID:25912189